{
  "gene_symbol": "SLC2A5",
  "gene_name": "Solute carrier family 2, facilitated glucose transporter member 5",
  "gene": "UniProtKB:P22732",
  "term_label": "D-glucose import",
  "term_id": "GO:0046323"
}